{
  "term_label": "RNA polymerase II cis-regulatory region sequence-specific DNA binding",
  "term_id": "GO:0000978",
  "gene_name": "Zinc finger and BTB domain-containing protein 22",
  "gene": "UniProtKB:O15209",
  "gene_symbol": "ZBTB22"
}